{
  "gene_name": "Forkhead box protein I2",
  "term_label": "RNA polymerase II cis-regulatory region sequence-specific DNA binding",
  "term_id": "GO:0000978",
  "gene": "UniProtKB:Q6ZQN5",
  "gene_symbol": "FOXI2"
}